MTREC complex binding [GO:1905763] (molecular function) References: PMID:26942678 Sources: GOC:TermGenie Also known as: Mtl1-Red1 core complex binding, NURS complex binding, PAXT complex binding Relationships: is a type of protein-containing complex binding [GO:0044877] Definition: Binding to a MTREC complex.